{
  "gene_name": "Keratin, type II cytoskeletal 2 oral",
  "term_label": "keratinization",
  "term_id": "GO:0031424",
  "gene_symbol": "KRT76",
  "gene": "UniProtKB:Q01546"
}